{
  "gene_symbol": "ARHGAP21",
  "term_id": "GO:0051645",
  "gene_name": "Rho GTPase-activating protein 21",
  "gene": "UniProtKB:Q5T5U3",
  "term_label": "Golgi localization"
}